{
  "term_id": "GO:0005759",
  "gene": "UniProtKB:Q969Z0",
  "term_label": "mitochondrial matrix",
  "gene_name": "FAST kinase domain-containing protein 4",
  "gene_symbol": "TBRG4"
}